{
  "gene_name": "Dixin",
  "term_label": "Unknown molecular function",
  "gene_symbol": "DIXDC1",
  "gene": "UniProtKB:Q155Q3",
  "term_id": "UNKNOWN:0001"
}